{
  "term_id": "GO:0046974",
  "term_label": "histone H3K9 methyltransferase activity",
  "gene_symbol": "SETDB2",
  "gene_name": "Histone-lysine N-methyltransferase SETDB2",
  "gene": "UniProtKB:Q96T68"
}